{
  "term_label": "defense response to Gram-negative bacterium",
  "term_id": "GO:0050829",
  "gene_symbol": "CAMP",
  "gene_name": "Cathelicidin antimicrobial peptide",
  "gene": "UniProtKB:P49913"
}